{
  "gene": "UniProtKB:Q96II8",
  "term_id": "GO:0005829",
  "gene_name": "DISP complex protein LRCH3",
  "term_label": "cytosol",
  "gene_symbol": "LRCH3"
}